{
  "term_id": "GO:0017147",
  "term_label": "Wnt-protein binding",
  "gene_symbol": "FZD7",
  "gene": "UniProtKB:O75084",
  "gene_name": "Frizzled-7"
}